{
  "term_id": "UNKNOWN:0002",
  "gene_name": "Oxysterol-binding protein-related protein 8",
  "gene_symbol": "OSBPL8",
  "gene": "UniProtKB:Q9BZF1",
  "term_label": "Unknown biological process"
}